{
  "gene": "UniProtKB:Q9GZR1",
  "term_id": "GO:0090234",
  "gene_name": "Sentrin-specific protease 6",
  "term_label": "regulation of kinetochore assembly",
  "gene_symbol": "SENP6"
}